termination of RNA polymerase II transcription, exosome-dependent [GO:0030847] (BP) Also known as: termination of RNA polymerase II transcription, poly(A)-independent, transcription termination from Pol II promoter, RNA polymerase(A)-independent, transcription termination from Pol II promoter, poly(A)-independent Relationships: is a type of termination of RNA polymerase II transcription [GO:0006369] References: PMID:12944462, PMID:18679429, PMID:27371117 Sources: GOC:txnOH Definition: The process in which transcription of nonpolyadenylated RNA polymerase II transcripts is terminated; coupled to the maturation of the RNA 3'-end.